{
  "term_label": "cellular response to calcium ion",
  "term_id": "GO:0071277",
  "gene": "UniProtKB:Q96FN4",
  "gene_symbol": "CPNE2",
  "gene_name": "Copine-2"
}